{
  "gene": "UniProtKB:Q9BTU6",
  "gene_symbol": "PI4K2A",
  "term_label": "trans-Golgi network",
  "gene_name": "Phosphatidylinositol 4-kinase type 2-alpha",
  "term_id": "GO:0005802"
}